{
  "term_id": "UNKNOWN:0001",
  "gene": "UniProtKB:P42166",
  "gene_name": "Lamina-associated polypeptide 2, isoform alpha",
  "term_label": "Unknown molecular function",
  "gene_symbol": "TMPO"
}